{
  "gene_name": "N-acetyllactosaminide beta-1,3-N-acetylglucosaminyltransferase 3",
  "gene_symbol": "B3GNT3",
  "term_label": "Golgi membrane",
  "term_id": "GO:0000139",
  "gene": "UniProtKB:Q9Y2A9"
}